substrate mycelium formation [GO:0097738] (biological process) References: PMID:10021365 Sources: GOC:di Relationships: is a type of anatomical structure development [GO:0048856]; is part of asexual reproduction [GO:0019954] Definition: The process by which, in some fungal species, hyphae grow as a network of invasive thread-like filaments formed from chains of attached cells within a solid or semi-solid substrate.